{
  "gene": "UniProtKB:Q8NAV1",
  "gene_symbol": "PRPF38A",
  "term_label": "Unknown biological process",
  "term_id": "UNKNOWN:0002",
  "gene_name": "Pre-mRNA-splicing factor 38A"
}